{
  "gene": "UniProtKB:A1L168",
  "gene_name": "Uncharacterized protein C20orf202",
  "term_label": "Unknown molecular function",
  "term_id": "UNKNOWN:0001",
  "gene_symbol": "C20orf202"
}